{
  "gene": "UniProtKB:P31641",
  "term_label": "taurine:sodium symporter activity",
  "gene_symbol": "SLC6A6",
  "term_id": "GO:0005369",
  "gene_name": "Sodium- and chloride-dependent taurine transporter"
}